{
  "gene": "UniProtKB:Q07325",
  "term_label": "neutrophil chemotaxis",
  "gene_name": "C-X-C motif chemokine 9",
  "term_id": "GO:0030593",
  "gene_symbol": "CXCL9"
}